{
  "gene_symbol": "CARD14",
  "term_id": "GO:0043123",
  "term_label": "positive regulation of canonical NF-kappaB signal transduction",
  "gene": "UniProtKB:Q9BXL6",
  "gene_name": "Caspase recruitment domain-containing protein 14"
}